{
  "gene_name": "Receptor-transporting protein 1",
  "term_label": "protein insertion into membrane",
  "gene": "UniProtKB:P59025",
  "gene_symbol": "RTP1",
  "term_id": "GO:0051205"
}